protein-glutathione oxidoreductase (glutathione) activity [GO:0141049] (molecular function) Also known as: glutaredoxin activity, glutathione oxidoreductase activity Relationships: is a type of disulfide oxidoreductase activity [GO:0015036]; is a type of oxidoreductase activity, acting on a sulfur group of donors, disulfide as acceptor [GO:0016671]; is a type of catalytic activity, acting on a protein [GO:0140096] Definition: Catalysis of the reaction: glutathionylated protein (PSSG) + glutathione (GSH) = protein-thiol (PSH) + glutathione disulfide (GSSG). The reaction may proceed via a 'monothiol' or 'dithiol' mechanism. References: PMID:23397885, PMID:33932870, PMID:36771108